{
  "term_label": "cell migration",
  "gene": "UniProtKB:Q9Y2A7",
  "gene_symbol": "NCKAP1",
  "term_id": "GO:0016477",
  "gene_name": "Nck-associated protein 1"
}